{
  "term_id": "GO:0005798",
  "gene": "UniProtKB:Q9UKJ5",
  "gene_symbol": "CHIC2",
  "gene_name": "Cysteine-rich hydrophobic domain-containing protein 2",
  "term_label": "Golgi-associated vesicle"
}